{
  "term_label": "nucleus",
  "gene_symbol": "STK35",
  "term_id": "GO:0005634",
  "gene": "UniProtKB:Q8TDR2",
  "gene_name": "Serine_threonine-protein kinase 35"
}